{
  "gene_name": "Protein FAM131A",
  "gene_symbol": "FAM131A",
  "term_id": "UNKNOWN:0002",
  "gene": "UniProtKB:Q6UXB0",
  "term_label": "Unknown biological process"
}